symbiont-mediated evasion of recognition by host pattern recognition receptor [GO:0141141] (biological process) Definition: A process by which a symbiont avoids recognition by host's innate immune response by altering or concealing a conserved molecule recognized by the host's cell surface and intracellular pattern recognition receptors, including Toll-like and NOD-like receptors. The host is defined as the larger of the organisms involved in a symbiotic interaction. Note: Note that this term should be used when the symbiont in cases where the symbiont modifies its own molecules (proteins, DNA, RNA, lipids) to avoid recognition by the host. In cases where the symbiont  directly inhibits a component of a host cytoplasmic receptor signaling pathway, consider annotating to evasion of symbiont recognition by host pattern recognition receptor ; GO:0039537. References: PMID:17215377, PMID:26502908, PMID:29101229 Relationships: is a type of GO:0141043 Also known as: evasion of symbiont recognition by host pattern recognition receptor